L-serine-pyruvate transaminase activity [GO:0004760] (MF) Definition: Catalysis of the reaction: L-serine + pyruvate = 3-hydroxypyruvate + L-alanine. Sources: EC:2.6.1.51, RHEA:22852 Also known as: serine-pyruvate aminotransferase activity, serine-pyruvate aminotransferase, type 1, serine-pyruvate aminotransferase, type 2A, serine-pyruvate aminotransferase, type 2B, L-serine:pyruvate aminotransferase activity, SPT, hydroxypyruvate:L-alanine transaminase activity, serine--pyruvate aminotransferase activity Relationships: is a type of transaminase activity [GO:0008483]